lysobisphosphatidic acid metabolic process [GO:2001311] (biological process) Also known as: LBPA metabolic process, LBPA metabolism, bis(monoacylglycerol) hydrogen phosphate (BMP) metabolic process, bis(monoacylglycerol) hydrogen phosphate (BMP) metabolism, bis(monoacylglycerol) hydrogen phosphate metabolic process, bis(monoacylglycerol) hydrogen phosphate metabolism, lysobisphosphatidic acid metabolism Definition: The chemical reactions and pathways involving a lysobisphosphatidic acid. A lysobisphosphatidic acid is a lysophosphatidic acid having the unusual property of a phosphodiester moiety linked to positions sn-1 and sn1' of glycerol; and two additional fatty acids esterified to the glycerol head group. Sources: GOC:mw Relationships: is a type of glycerophospholipid metabolic process [GO:0006650]; is a type of alditol phosphate metabolic process [GO:0052646] Subtypes: lysobisphosphatidic acid biosynthetic process [GO:2001312]